{
  "term_id": "GO:0006621",
  "gene_symbol": "KDELR2",
  "gene": "UniProtKB:P33947",
  "gene_name": "ER lumen protein-retaining receptor 2",
  "term_label": "protein retention in ER lumen"
}